{
  "term_id": "UNKNOWN:0001",
  "gene_name": "Putative uncharacterized protein PRO3102",
  "gene": "UniProtKB:Q9H379",
  "gene_symbol": "PRO3102",
  "term_label": "Unknown molecular function"
}